L-fucose isomerase activity [GO:0008736] (molecular function) Also known as: L-fucose aldose-ketose-isomerase activity, L-fucose ketol-isomerase activity Sources: RHEA:17233 Definition: Catalysis of the reaction: L-fucose = L-fuculose. Relationships: is a type of intramolecular oxidoreductase activity, interconverting aldoses and ketoses [GO:0016861]